{
  "gene_symbol": "KCNN1",
  "term_label": "small conductance calcium-activated potassium channel activity",
  "gene_name": "Small conductance calcium-activated potassium channel protein 1",
  "term_id": "GO:0016286",
  "gene": "UniProtKB:Q92952"
}